vistamycin catabolic process [GO:1901151] (biological process) Definition: The chemical reactions and pathways resulting in the breakdown of vistamycin. Also known as: ribostamycin breakdown, ribostamycin catabolic process, ribostamycin catabolism, ribostamycin degradation, vistamycin breakdown, vistamycin catabolism, vistamycin degradation Sources: GOC:TermGenie, GOC:yaf, UniPathway:UPA00972 Relationships: is a type of GO:0030649; is a type of polyol catabolic process [GO:0046174]